{
  "term_id": "UNKNOWN:0001",
  "gene": "UniProtKB:Q9NRS6",
  "gene_name": "Sorting nexin-15",
  "gene_symbol": "SNX15",
  "term_label": "Unknown molecular function"
}